{
  "gene": "UniProtKB:O00194",
  "term_id": "GO:0030141",
  "gene_symbol": "RAB27B",
  "gene_name": "Ras-related protein Rab-27B",
  "term_label": "secretory granule"
}